{
  "term_id": "GO:0051896",
  "gene": "UniProtKB:Q9UBG3",
  "gene_name": "Cornulin",
  "gene_symbol": "CRNN",
  "term_label": "regulation of phosphatidylinositol 3-kinase/protein kinase B signal transduction"
}